{
  "term_label": "Unknown cellular component",
  "term_id": "UNKNOWN:0003",
  "gene_name": "Atypical kinase COQ8A, mitochondrial",
  "gene": "UniProtKB:Q8NI60",
  "gene_symbol": "COQ8A"
}